positive regulation of termination of RNA polymerase I transcription [GO:2000732] (biological process) Also known as: positive regulation of RNA polymerase I transcription termination, positive regulation of transcription termination from Pol I promoter, positive regulation of transcription termination from RNA polymerase I promoter Sources: GOC:obol Definition: Any process that activates or increases the frequency, rate or extent of termination of RNA polymerase I transcription. Relationships: is a type of positive regulation of transcription by RNA polymerase I [GO:0045943]; is a type of positive regulation of termination of DNA-templated transcription [GO:0060566]; is a type of GO:2000730; positively regulates GO:0006363